dTDP-4-amino-4,6-dideoxygalactose transaminase activity [GO:0019180] (molecular function) Sources: EC:2.6.1.59, RHEA:10368 Also known as: dTDP-fucosamine aminotransferase activity, dTDP-4,6-dideoxy-D-galactose:2-oxoglutarate aminotransferase activity, dTDP-4-amino-4,6-dideoxygalactose aminotransferase activity, thymidine diphosphate 4-keto-6-deoxy-D-glucose transaminase activity, thymidine diphosphoaminodideoxygalactose aminotransferase activity Relationships: is_a transaminase activity [GO:0008483] Definition: Catalysis of the reaction: 2-oxoglutarate + dTDP-4-amino-4,6-dideoxy-D-galactose = L-glutamate + dTDP-4-dehydro-6-deoxy-D-galactose.